{
  "term_label": "maintenance of synapse structure",
  "gene_name": "C1q-related factor",
  "gene_symbol": "C1QL1",
  "term_id": "GO:0099558",
  "gene": "UniProtKB:O75973"
}